{
  "gene": "UniProtKB:Q9UHP3",
  "gene_name": "Ubiquitin carboxyl-terminal hydrolase 25",
  "gene_symbol": "USP25",
  "term_label": "nucleus",
  "term_id": "GO:0005634"
}